{
  "term_id": "UNKNOWN:0001",
  "gene": "UniProtKB:P60602",
  "term_label": "Unknown molecular function",
  "gene_name": "Reactive oxygen species modulator 1",
  "gene_symbol": "ROMO1"
}